{
  "gene_symbol": "EIF1B",
  "gene_name": "Eukaryotic translation initiation factor 1b",
  "term_label": "translation initiation factor activity",
  "gene": "UniProtKB:O60739",
  "term_id": "GO:0003743"
}